{
  "term_label": "cytoplasm",
  "term_id": "GO:0005737",
  "gene": "UniProtKB:A0MZ66",
  "gene_symbol": "SHTN1",
  "gene_name": "Shootin-1"
}